alpha-catenin binding [GO:0045294] (MF) Definition: Binding to catenin complex alpha subunit. Sources: GOC:bf Relationships: is a type of GO:0005515